{
  "gene_symbol": "XKR5",
  "gene": "UniProtKB:Q6UX68",
  "term_label": "Unknown molecular function",
  "term_id": "UNKNOWN:0001",
  "gene_name": "XK-related protein 5"
}